{
  "gene_name": "Leucine-rich repeat and death domain-containing protein 1",
  "gene": "UniProtKB:A4D1F6",
  "term_label": "Unknown biological process",
  "gene_symbol": "LRRD1",
  "term_id": "UNKNOWN:0002"
}